{
  "term_label": "protein folding",
  "gene_symbol": "PPIF",
  "term_id": "GO:0006457",
  "gene_name": "Peptidyl-prolyl cis-trans isomerase F, mitochondrial",
  "gene": "UniProtKB:P30405"
}